3-hydroxybenzoate 6-monooxygenase activity [GO:0018669] (molecular function) Sources: EC:1.14.13.24, RHEA:22692 Relationships: is a type of GO:0016709 Definition: Catalysis of the reaction: 3-hydroxybenzoate + H+ + NADH + O2 = 2,5-dihydroxybenzoate + H2O + NAD+. Also known as: 3-hydroxybenzoate 6-hydroxylase activity, 3-hydroxybenzoate,NADH:oxygen oxidoreductase (6-hydroxylating), 3-hydroxybenzoic acid-6-hydroxylase activity, m-hydroxybenzoate 6-hydroxylase activity